acetoin racemase activity [GO:0047604] (molecular function) Also known as: acetylmethylcarbinol racemase activity Sources: EC:5.1.2.4, RHEA:12092 Definition: Catalysis of the reaction: (S)-acetoin = (R)-acetoin. Relationships: is a type of racemase and epimerase activity, acting on hydroxy acids and derivatives [GO:0016856]